negative regulation of hydrogen peroxide metabolic process [GO:0010727] (biological process) Subtypes: negative regulation of hydrogen peroxide biosynthetic process [GO:0010730], negative regulation of hydrogen peroxide catabolic process [GO:2000296] Relationships: is_a regulation of hydrogen peroxide metabolic process [GO:0010310]; is a type of negative regulation of reactive oxygen species metabolic process [GO:2000378]; negatively regulates hydrogen peroxide metabolic process [GO:0042743] Definition: Any process that decreases the frequency, rate or extent of the chemical reactions and pathways involving hydrogen peroxide. Sources: GOC:dph, GOC:hjd, GOC:tb Also known as: negative regulation of hydrogen peroxide metabolism